5.8S rRNA binding [GO:1990932] (molecular function) Definition: Binding to 5.8S ribosomal RNA, a eukaryotic ribosomal RNA which forms a complex with 28S RNA. References: PMID:11716358, PMID:15527424 Relationships: is a type of rRNA binding [GO:0019843]